{
  "gene_symbol": "OTULINL",
  "term_id": "UNKNOWN:0001",
  "gene": "UniProtKB:Q9NUU6",
  "term_label": "Unknown molecular function",
  "gene_name": "Inactive ubiquitin thioesterase OTULINL"
}